trans-synaptic signaling by nitric oxide, modulating synaptic transmission [GO:0099555] (biological process) Definition: Cell-cell signaling between presynapse and postsynapse, via the release and reception of nitric oxide molecules, that modulates the synaptic transmission properties of the synapse. Sources: GOC:dos Note: Note that this term was created for the SynGO project, and will be obsoleted when the SynGO annotations are made in Noctua. Relationships: is a type of trans-synaptic signaling by nitric oxide [GO:0099548]; is a type of trans-synaptic signaling by soluble gas, modulating synaptic transmission [GO:0099554] Subtypes: retrograde trans-synaptic signaling by nitric oxide, modulating synaptic transmission [GO:0098925]